{
  "term_label": "Unknown molecular function",
  "gene_symbol": "MITD1",
  "gene_name": "MIT domain-containing protein 1",
  "term_id": "UNKNOWN:0001",
  "gene": "UniProtKB:Q8WV92"
}